{
  "gene": "UniProtKB:Q9UER7",
  "term_id": "GO:0006334",
  "gene_symbol": "DAXX",
  "gene_name": "Death domain-associated protein 6",
  "term_label": "nucleosome assembly"
}